{
  "term_label": "cytosol",
  "gene_symbol": "PSMD13",
  "gene": "UniProtKB:Q9UNM6",
  "term_id": "GO:0005829",
  "gene_name": "26S proteasome non-ATPase regulatory subunit 13"
}